{
  "term_id": "GO:0004951",
  "gene": "UniProtKB:P32238",
  "term_label": "cholecystokinin receptor activity",
  "gene_symbol": "CCKAR",
  "gene_name": "Cholecystokinin receptor type A"
}